{
  "term_label": "animal organ morphogenesis",
  "term_id": "GO:0009887",
  "gene_name": "Putative Polycomb group protein ASXL2",
  "gene": "UniProtKB:Q76L83",
  "gene_symbol": "ASXL2"
}